negative regulation of cellular response to phosphate starvation [GO:0140256] (BP) Definition: Any process that stops, prevents or reduces the frequency, rate or extent of cellular response to phosphate starvation. References: PMID:29414789 Relationships: is a type of negative regulation of response to nutrient levels [GO:0032108]; is a type of negative regulation of cellular process [GO:0048523]; is a type of GO:0140255; negatively regulates GO:0016036